{
  "term_id": "GO:0000978",
  "gene_name": "Circadian-associated transcriptional repressor",
  "gene_symbol": "CIART",
  "term_label": "RNA polymerase II cis-regulatory region sequence-specific DNA binding",
  "gene": "UniProtKB:Q8N365"
}